regulation of mitotic division septum assembly [GO:0140279] (biological process) Subtypes: negative regulation of mitotic division septum assembly [GO:0140280], GO:0140281, regulation of primary cell septum biogenesis [GO:1905756] Definition: Any process that modulates the frequency, rate or extent of mitotic division septum formation. Division septum formation is the assembly and arrangement of a septum that spans the plasma membrane interface between progeny cells following cytokinesis. References: PMID:22786806 Relationships: is a type of regulation of division septum assembly [GO:0032955]; is a type of GO:1903436; regulates GO:0140278 Also known as: regulation of division septum formation involved in mitotic cell cycle, regulation of formation of division septum involved in mitotic cell cycle, regulation of septin assembly and septum biosynthesis involved in mitotic cell cycle, regulation of septin assembly and septum formation involved in mitotic cell cycle